negative regulation of extrinsic apoptotic signaling pathway via death domain receptors [GO:1902042] (biological process) Relationships: is a type of GO:1902041; is a type of negative regulation of extrinsic apoptotic signaling pathway [GO:2001237]; negatively regulates extrinsic apoptotic signaling pathway via death domain receptors [GO:0008625] Also known as: down regulation of extrinsic apoptotic signaling pathway via death domain receptors, down-regulation of extrinsic apoptotic signaling pathway via death domain receptors, downregulation of extrinsic apoptotic signaling pathway via death domain receptors, down regulation of death receptor-mediated apoptosis, down-regulation of death receptor-mediated apoptosis, downregulation of death receptor-mediated apoptosis, inhibition of death receptor-mediated apoptosis, inhibition of extrinsic apoptotic signaling pathway via death domain receptors, negative regulation of death receptor-mediated apoptosis References: PMID:17245429 Sources: GOC:TermGenie Subtypes: negative regulation of TRAIL-activated apoptotic signaling pathway [GO:1903122] Definition: Any process that stops, prevents or reduces the frequency, rate or extent of extrinsic apoptotic signaling pathway via death domain receptors.